{
  "term_id": "GO:0030246",
  "term_label": "carbohydrate binding",
  "gene_name": "C-type lectin domain family 4 member G",
  "gene": "UniProtKB:Q6UXB4",
  "gene_symbol": "CLEC4G"
}